2-dehydro-3-deoxyglucarate aldolase activity [GO:0008672] (molecular function) Sources: EC:4.1.2.20 Definition: Catalysis of the reaction: 2-dehydro-3-deoxy-D-glucarate = pyruvate + tartronate semialdehyde. Also known as: 2-dehydro-3-deoxy-D-glucarate tartronate-semialdehyde-lyase (pyruvate-forming), 2-dehydro-3-deoxy-D-glucarate tartronate-semialdehyde-lyase activity, 2-keto-3-deoxyglucarate aldolase activity, alpha-keto-beta-deoxy-D-glucarate aldolase activity Relationships: is a type of GO:0016832